{
  "gene": "UniProtKB:P49281",
  "gene_symbol": "SLC11A2",
  "gene_name": "Natural resistance-associated macrophage protein 2",
  "term_label": "endosome membrane",
  "term_id": "GO:0010008"
}